orlandin metabolic process [GO:1900819] (biological process) Definition: The chemical reactions and pathways involving orlandin. Sources: GOC:TermGenie, GOC:di Subtypes: GO:1900820, orlandin biosynthetic process [GO:1900821] Relationships: is a type of secondary metabolic process [GO:0019748] Also known as: orlandin metabolism